{
  "term_label": "Unknown biological process",
  "term_id": "UNKNOWN:0002",
  "gene_symbol": "PRDM7",
  "gene_name": "Histone-lysine N-methyltransferase PRDM7",
  "gene": "UniProtKB:Q9NQW5"
}